{
  "gene": "UniProtKB:Q16548",
  "term_label": "extrinsic apoptotic signaling pathway in absence of ligand",
  "term_id": "GO:0097192",
  "gene_name": "Bcl-2-related protein A1",
  "gene_symbol": "BCL2A1"
}